{
  "term_id": "GO:0006637",
  "gene_name": "Peroxisomal succinyl-coenzyme A thioesterase",
  "term_label": "acyl-CoA metabolic process",
  "gene_symbol": "ACOT4",
  "gene": "UniProtKB:Q8N9L9"
}